{
  "gene_name": "C2 domain-containing protein 5",
  "term_id": "GO:0010828",
  "term_label": "positive regulation of D-glucose transmembrane transport",
  "gene": "UniProtKB:Q86YS7",
  "gene_symbol": "C2CD5"
}